{
  "term_label": "interleukin-18-mediated signaling pathway",
  "gene_name": "Interleukin-18",
  "gene_symbol": "IL18",
  "gene": "UniProtKB:Q14116",
  "term_id": "GO:0035655"
}